{
  "term_id": "GO:0000981",
  "gene_symbol": "ZNF137P",
  "term_label": "DNA-binding transcription factor activity, RNA polymerase II-specific",
  "gene_name": "Putative zinc finger protein 137",
  "gene": "UniProtKB:P52743"
}